viral DNA genome packaging [GO:0019073] (biological process) Sources: ISBN:0781702534 Subtypes: GO:0098006, viral DNA genome packaging via site-specific sequence recognition [GO:0098035] Relationships: is a type of GO:0019072 Definition: The packing of viral DNA into a capsid.